{
  "gene_symbol": "TRAV14DV4",
  "term_id": "UNKNOWN:0001",
  "gene_name": "T cell receptor alpha variable 14_delta variable 4",
  "gene": "UniProtKB:A0A0A6YYC5",
  "term_label": "Unknown molecular function"
}